{
  "term_id": "UNKNOWN:0002",
  "gene_name": "Solute carrier family 25 member 48",
  "gene_symbol": "SLC25A48",
  "gene": "UniProtKB:Q6ZT89",
  "term_label": "Unknown biological process"
}